{
  "gene_symbol": "ANKS1A",
  "gene_name": "Ankyrin repeat and SAM domain-containing protein 1A",
  "term_id": "GO:0048013",
  "gene": "UniProtKB:Q92625",
  "term_label": "ephrin receptor signaling pathway"
}